{
  "gene_symbol": "REG3A",
  "gene_name": "Regenerating islet-derived protein 3-alpha",
  "term_id": "GO:0005615",
  "term_label": "extracellular space",
  "gene": "UniProtKB:Q06141"
}